{
  "term_label": "protein kinase binding",
  "gene": "UniProtKB:A6NLX3",
  "term_id": "GO:0019901",
  "gene_name": "Speedy protein E4",
  "gene_symbol": "SPDYE4"
}